{
  "term_id": "GO:0005886",
  "gene_symbol": "FRMD8P1",
  "gene": "UniProtKB:Q9BZ68",
  "term_label": "plasma membrane",
  "gene_name": "Putative FERM domain-containing protein FRMD8P1"
}